{
  "gene": "UniProtKB:P30048",
  "gene_name": "Thioredoxin-dependent peroxide reductase, mitochondrial",
  "term_label": "thioredoxin peroxidase activity",
  "gene_symbol": "PRDX3",
  "term_id": "GO:0008379"
}